{
  "gene_name": "B melanoma antigen 1",
  "gene_symbol": "BAGE",
  "term_label": "Unknown molecular function",
  "term_id": "UNKNOWN:0001",
  "gene": "UniProtKB:Q13072"
}